negative regulation of ascospore formation [GO:0075297] (BP) Sources: GOC:pamgo_curators Relationships: is a type of GO:0010721; is_a negative regulation of cell cycle process [GO:0010948]; is a type of regulation of ascospore formation [GO:0034307]; is a type of negative regulation of sexual sporulation resulting in formation of a cellular spore [GO:0043942]; negatively regulates ascospore formation [GO:0030437] Definition: Any process that stops, prevents, or reduces the frequency, rate or extent of ascospore formation, a process in which a sexual spore, named ascospore, from Ascomycete fungi was produced inside an ascus.